{
  "gene": "UniProtKB:Q9BSU3",
  "gene_symbol": "NAA11",
  "term_label": "protein N-terminal-serine acetyltransferase activity",
  "gene_name": "N-alpha-acetyltransferase 11",
  "term_id": "GO:1990189"
}